{
  "term_id": "GO:0009725",
  "gene_symbol": "TIMP4",
  "gene": "UniProtKB:Q99727",
  "term_label": "response to hormone",
  "gene_name": "Metalloproteinase inhibitor 4"
}